{
  "gene_symbol": "ST18",
  "term_label": "regulation of gene expression",
  "term_id": "GO:0010468",
  "gene_name": "Suppression of tumorigenicity 18 protein",
  "gene": "UniProtKB:O60284"
}